{
  "gene": "UniProtKB:P39880",
  "gene_symbol": "CUX1",
  "term_label": "nucleus",
  "term_id": "GO:0005634",
  "gene_name": "Homeobox protein cut-like 1"
}